{
  "gene_name": "Uncharacterized protein C15orf61",
  "term_id": "UNKNOWN:0001",
  "gene": "UniProtKB:A6NNL5",
  "term_label": "Unknown molecular function",
  "gene_symbol": "C15orf61"
}